{
  "term_label": "Unknown biological process",
  "gene_symbol": "NOTCH2NLR",
  "gene": "UniProtKB:A0A096LNW5",
  "term_id": "UNKNOWN:0002",
  "gene_name": "Notch homolog 2 N-terminal-like protein R"
}